{
  "term_id": "GO:0000774",
  "gene_name": "BAG family molecular chaperone regulator 5",
  "term_label": "adenyl-nucleotide exchange factor activity",
  "gene_symbol": "BAG5",
  "gene": "UniProtKB:Q9UL15"
}